{
  "term_label": "transcription factor TFIIE complex",
  "term_id": "GO:0005673",
  "gene_name": "General transcription factor IIE subunit 1",
  "gene": "UniProtKB:P29083",
  "gene_symbol": "GTF2E1"
}